{
  "gene_symbol": "DPY30",
  "gene_name": "Protein dpy-30 homolog",
  "term_label": "Unknown biological process",
  "term_id": "UNKNOWN:0002",
  "gene": "UniProtKB:Q9C005"
}